{
  "gene_name": "Ornithine decarboxylase antizyme 1",
  "gene": "UniProtKB:P54368",
  "term_label": "Unknown biological process",
  "term_id": "UNKNOWN:0002",
  "gene_symbol": "OAZ1"
}